{
  "term_id": "UNKNOWN:0003",
  "term_label": "Unknown cellular component",
  "gene": "UniProtKB:A0A1B0GUZ9",
  "gene_name": "Uncharacterized protein",
  "gene_symbol": "A0A1B0GUZ9"
}